response to paraquat [GO:1901562] (biological process) Sources: GOC:TermGenie Definition: Any process that results in a change in state or activity of a cell or an organism (in terms of movement, secretion, enzyme production, gene expression, etc.) as a result of a paraquat stimulus. Subtypes: cellular response to paraquat [GO:0072756] Relationships: is a type of GO:0042221